{
  "term_label": "cytoplasm",
  "gene_name": "Leucine-rich repeat and IQ domain-containing protein 4",
  "gene": "UniProtKB:A6NIV6",
  "gene_symbol": "LRRIQ4",
  "term_id": "GO:0005737"
}